{
  "term_label": "chemical synaptic transmission",
  "term_id": "GO:0007268",
  "gene": "UniProtKB:Q16572",
  "gene_name": "Vesicular acetylcholine transporter",
  "gene_symbol": "SLC18A3"
}